small-subunit processome [GO:0032040] (cellular component) Relationships: is a type of preribosome [GO:0030684]; is a type of GO:0140513; BFO_0000050 nucleolus [GO:0005730]; has part t-UTP complex [GO:0034455] References: PMID:12068309, PMID:12957375, PMID:15120992, PMID:15590835 Sources: GOC:krc, GOC:vw Definition: A large ribonucleoprotein complex that is an early preribosomal complex. In S. cerevisiae, it has a size of 80S and consists of the 35S pre-rRNA, early-associating ribosomal proteins most of which are part of the small ribosomal subunit, the U3 snoRNA and associated proteins. Also known as: SSU processome, small subunit processome